{
  "term_id": "GO:0019722",
  "gene_symbol": "CCR3",
  "gene": "UniProtKB:P51677",
  "gene_name": "C-C chemokine receptor type 3",
  "term_label": "calcium-mediated signaling"
}